{
  "gene": "UniProtKB:Q9BSF0",
  "term_id": "UNKNOWN:0002",
  "term_label": "Unknown biological process",
  "gene_name": "Small membrane A-kinase anchor protein",
  "gene_symbol": "C2orf88"
}